{
  "term_label": "cytosol",
  "gene_name": "G-protein coupled receptor-associated sorting protein 1",
  "gene_symbol": "GPRASP1",
  "term_id": "GO:0005829",
  "gene": "UniProtKB:Q5JY77"
}